{
  "gene_name": "Secreted frizzled-related protein 1",
  "gene": "UniProtKB:Q8N474",
  "term_id": "GO:0035567",
  "term_label": "non-canonical Wnt signaling pathway",
  "gene_symbol": "SFRP1"
}